kainate selective glutamate receptor activity [GO:0015277] (molecular function) Definition: An ionotropic glutamate receptor activity that exhibits fast gating by glutamate, acts by opening a cation channel permeable to sodium and potassium, and for which kainate is an agonist. References: PMID:10049997, PMID:8804111 Sources: GOC:mah Note: Note that this term represents an activity and not a gene product. Consider also annotating to the molecular function terms 'ionotropic glutamate receptor activity ; GO:0004970' and 'cation channel activity ; GO:0005261'. Relationships: is a type of glutamate-gated receptor activity [GO:0004970]; is a type of potassium channel activity [GO:0005267]; is a type of ligand-gated sodium channel activity [GO:0015280]